{
  "term_id": "GO:0038023",
  "gene_name": "Membrane progestin receptor delta",
  "gene_symbol": "PAQR6",
  "term_label": "signaling receptor activity",
  "gene": "UniProtKB:Q6TCH4"
}